{
  "gene_name": "ER membrane protein complex subunit 8",
  "gene": "UniProtKB:O43402",
  "gene_symbol": "EMC8",
  "term_id": "GO:0045050",
  "term_label": "protein insertion into ER membrane by stop-transfer membrane-anchor sequence"
}